{
  "gene_symbol": "NR2F1",
  "term_label": "nuclear receptor activity",
  "term_id": "GO:0004879",
  "gene_name": "COUP transcription factor 1",
  "gene": "UniProtKB:P10589"
}